{
  "term_id": "GO:0005634",
  "gene": "UniProtKB:P35398",
  "gene_name": "Nuclear receptor ROR-alpha",
  "gene_symbol": "RORA",
  "term_label": "nucleus"
}